{
  "term_label": "spindle organization",
  "gene": "UniProtKB:Q9NQ86",
  "gene_name": "E3 ubiquitin-protein ligase TRIM36",
  "gene_symbol": "TRIM36",
  "term_id": "GO:0007051"
}